style development [GO:0048479] (biological process) Relationships: is a type of developmental process involved in reproduction [GO:0003006]; is a type of anatomical structure development [GO:0048856]; is part of carpel development [GO:0048440] Sources: GOC:jid, PO:0009074 Definition: The process whose specific outcome is the progression of the style over time, from its formation to the mature structure. The style is an elongated part of a carpel, or group of fused carpels, and it lies between the ovary and the stigma.